{
  "gene_name": "Heat shock protein HSP 90-alpha A2",
  "term_label": "ATP hydrolysis activity",
  "gene": "UniProtKB:Q14568",
  "gene_symbol": "HSP90AA2P",
  "term_id": "GO:0016887"
}